response to meiotic spindle assembly checkpoint signaling [GO:0072464] (biological process) Definition: A process that occurs in response to signals generated as a result of meiotic spindle assembly checkpoint signaling. Sources: GOC:mtg_cell_cycle Relationships: is a type of response to meiotic cell cycle checkpoint signaling [GO:0072410]; is_a response to spindle assembly checkpoint signaling [GO:0072485] Also known as: meiotic spindle assembly checkpoint effector process, response to signal involved in meiotic spindle assembly checkpoint